{
  "term_label": "lipase binding",
  "gene_symbol": "GPIHBP1",
  "gene": "UniProtKB:Q8IV16",
  "term_id": "GO:0035473",
  "gene_name": "Glycosylphosphatidylinositol-anchored high density lipoprotein-binding protein 1"
}